protein import into peroxisome matrix, docking [GO:0016560] (biological process) Relationships: is a type of intracellular protein localization [GO:0008104]; is part of GO:0016558 References: PMID:11687502, PMID:11988772, PMID:14754507 Definition: The process in which a complex formed of a peroxisome targeting sequence (PTS) receptor bound to a PTS-bearing protein docks with translocation machinery in the peroxisomal membrane. Also known as: peroxisome matrix protein import, docking, protein docking during peroxisome matrix protein import, protein docking during protein import into peroxisome matrix, protein docking during protein transport into peroxisome matrix, protein transport into peroxisome matrix, docking, peroxisome receptor docking